{
  "gene": "UniProtKB:Q9NQG1",
  "term_id": "UNKNOWN:0001",
  "gene_name": "Protein MANBAL",
  "term_label": "Unknown molecular function",
  "gene_symbol": "MANBAL"
}